{
  "term_label": "Unknown cellular component",
  "gene": "UniProtKB:A6NI47",
  "term_id": "UNKNOWN:0003",
  "gene_symbol": "POTEM",
  "gene_name": "Putative POTE ankyrin domain family member M"
}